{
  "term_label": "synaptic vesicle endocytosis",
  "gene_name": "Gamma-synuclein",
  "gene": "UniProtKB:O76070",
  "gene_symbol": "SNCG",
  "term_id": "GO:0048488"
}